morphogenesis of a branching epithelium [GO:0061138] (biological process) Sources: GOC:dph Definition: The process in which the anatomical structures of a branched epithelium are generated and organized. Relationships: is a type of GO:0001763; is a type of morphogenesis of an epithelium [GO:0002009] Subtypes: branching morphogenesis of an epithelial tube [GO:0048754], branching involved in prostate gland morphogenesis [GO:0060442], branching involved in salivary gland morphogenesis [GO:0060445], GO:0060670, branching involved in pancreas morphogenesis [GO:0061114], GO:0061683